{
  "term_label": "insulin catabolic process",
  "term_id": "GO:1901143",
  "gene_name": "Chymotrypsin-like elastase family member 2B",
  "gene_symbol": "CELA2B",
  "gene": "UniProtKB:P08218"
}